hippocampal interneuron differentiation [GO:0097410] (biological process) Definition: The process in which a relatively unspecialized cell acquires specialized features of a hippocampal interneuron. References: PMID:19655320 Sources: CL:1001569, GOC:jc Relationships: is a type of cerebral cortex neuron differentiation [GO:0021895]; is part of GO:0021766